{
  "gene_name": "Protein FAM124A",
  "term_id": "UNKNOWN:0002",
  "gene_symbol": "FAM124A",
  "gene": "UniProtKB:Q86V42",
  "term_label": "Unknown biological process"
}